{
  "term_label": "endoplasmic reticulum",
  "term_id": "GO:0005783",
  "gene": "UniProtKB:Q86SQ9",
  "gene_name": "Dehydrodolichyl diphosphate synthase complex subunit DHDDS",
  "gene_symbol": "DHDDS"
}